endodermal digestive tract morphogenesis [GO:0061031] (biological process) Sources: GOC:dph, GOC:yaf Relationships: is a type of digestive tract morphogenesis [GO:0048546] Definition: The process in which the anatomical structures of the endodermal digestive tract are generated and organized. The endodermal digestive tract includes those portions of the digestive tract that are derived from endoderm.